{
  "gene_name": "Neurogenin-2",
  "gene_symbol": "NEUROG2",
  "gene": "UniProtKB:Q9H2A3",
  "term_id": "GO:0000981",
  "term_label": "DNA-binding transcription factor activity, RNA polymerase II-specific"
}